regulation of neurotransmitter receptor localization to postsynaptic specialization membrane [GO:0098696] (biological process) Relationships: is a type of regulation of biological quality [GO:0065008]; is a type of GO:1902473; is a type of regulation of receptor localization to synapse [GO:1902683]; is a type of regulation of protein localization to cell periphery [GO:1904375]; is a type of regulation of protein localization to membrane [GO:1905475]; regulates GO:0099645 Definition: Any process that modulates the frequency, rate or extent of neurotransmitter receptor localization to postsynaptic specialization membrane. Sources: GOC:dos